{
  "gene_symbol": "MARCHF1",
  "gene": "UniProtKB:Q8TCQ1",
  "term_id": "GO:0000209",
  "term_label": "protein polyubiquitination",
  "gene_name": "E3 ubiquitin-protein ligase MARCHF1"
}